negative regulation of lipoprotein oxidation [GO:0034443] (biological process) Definition: Any process that stops, prevents, or reduces the frequency, rate or extent of lipoprotein oxidation. Also known as: inhibition of lipoprotein oxidation Sources: GOC:BHF, GOC:mah Relationships: is_a regulation of lipoprotein oxidation [GO:0034442]; is a type of GO:0050748; negatively regulates lipoprotein oxidation [GO:0042161] Subtypes: negative regulation of lipoprotein lipid oxidation [GO:0060588]